positive regulation of neutrophil degranulation [GO:0043315] (biological process) Definition: Any process that activates or increases the frequency, rate or extent of neutrophil degranulation. Sources: ISBN:0781735149 Also known as: positive regulation of neutrophil granule exocytosis, up regulation of neutrophil degranulation, up-regulation of neutrophil degranulation, upregulation of neutrophil degranulation, activation of neutrophil degranulation, stimulation of neutrophil degranulation Relationships: is a type of positive regulation of myeloid leukocyte mediated immunity [GO:0002888]; is a type of positive regulation of leukocyte degranulation [GO:0043302]; is a type of regulation of neutrophil degranulation [GO:0043313]; is a type of positive regulation of immune response [GO:0050778]; positively regulates neutrophil degranulation [GO:0043312]